{
  "gene_name": "RAD52 motif-containing protein 1",
  "gene_symbol": "RDM1",
  "term_label": "nucleolus",
  "gene": "UniProtKB:Q8NG50",
  "term_id": "GO:0005730"
}